{
  "gene_name": "Tetraspanin-17",
  "term_label": "plasma membrane",
  "gene_symbol": "TSPAN17",
  "gene": "UniProtKB:Q96FV3",
  "term_id": "GO:0005886"
}